{
  "gene": "UniProtKB:Q9BZG2",
  "gene_symbol": "ACP4",
  "gene_name": "Testicular acid phosphatase",
  "term_id": "GO:0120154",
  "term_label": "negative regulation of ERBB4 signaling pathway"
}